negative regulation of Arp2/3 complex-mediated actin nucleation [GO:0034316] (biological process) Relationships: is a type of GO:0034315; is_a negative regulation of actin nucleation [GO:0051126]; negatively regulates Arp2/3 complex-mediated actin nucleation [GO:0034314] References: PMID:16959963 Sources: GOC:mah Definition: Any process that stops, prevents, or reduces the frequency, rate or extent of actin nucleation mediated by the Arp2/3 complex and interacting proteins.